{
  "gene": "UniProtKB:Q99731",
  "gene_symbol": "CCL19",
  "term_id": "GO:0061844",
  "term_label": "antimicrobial humoral immune response mediated by antimicrobial peptide",
  "gene_name": "C-C motif chemokine 19"
}